{
  "gene_name": "Syntaxin-17",
  "gene": "UniProtKB:P56962",
  "term_label": "vesicle docking",
  "term_id": "GO:0048278",
  "gene_symbol": "STX17"
}